regulation of neosartoricin biosynthetic process [GO:1902053] (biological process) Subtypes: GO:1902054, positive regulation of neosartoricin biosynthetic process [GO:1902055] References: PMID:23368997 Sources: GOC:TermGenie, GOC:di Relationships: is a type of regulation of polyketide biosynthetic process [GO:1900732]; is a type of regulation of alcohol biosynthetic process [GO:1902930]; regulates GO:1902050 Also known as: regulation of neosartoricin anabolism, regulation of neosartoricin biosynthesis, regulation of neosartoricin formation, regulation of neosartoricin synthesis Definition: Any process that modulates the frequency, rate or extent of neosartoricin biosynthetic process.